{
  "gene": "UniProtKB:Q8IWF2",
  "gene_name": "FAD-dependent oxidoreductase domain-containing protein 2",
  "term_label": "monooxygenase activity",
  "term_id": "GO:0004497",
  "gene_symbol": "FOXRED2"
}